vulval location [GO:0034608] (biological process) Definition: Location, by the male, of his partner's vulva when backing along the ventral side of the hermaphrodite during mating. The male stops at the vulva, coordinates his movements to the hermaphrodite's, and positions his tail precisely over the vulva so that he may insert his spicules and ejaculate. References: PMID:18050467 Relationships: is_a GO:0060179